NAD(P)H dehydrogenase (quinone) activity [GO:0003955] (molecular function) Sources: EC:1.6.5.2 Relationships: is a type of oxidoreductase activity, acting on NAD(P)H, quinone or similar compound as acceptor [GO:0016655] Definition: Catalysis of the reaction: NAD(P)H + H+ + a quinone = NAD(P)+ + a quinol. Also known as: NAD(P)H dehydrogenase activity, NAD(P)H menadione reductase activity, NAD(P)H: menadione oxidoreductase activity, azoreductase activity, diaphorase activity, NADH-menadione reductase activity, menadione oxidoreductase activity, menadione reductase activity, naphthoquinone reductase activity, p-benzoquinone reductase activity, phylloquinone reductase activity, viologen accepting pyridine nucleotide oxidoreductase activity, vitamin K reductase activity, vitamin-K reductase activity, DT-diaphorase activity, NAD(P)H(2) dehydrogenase (quinone) activity, NAD(P)H-quinone dehydrogenase activity, NAD(P)H-quinone oxidoreductase activity, NAD(P)H2 dehydrogenase (quinone), NAD(P)H:(quinone-acceptor)oxidoreductase activity, NAD(P)H:quinone oxidoreductase activity, NQO1, QR1, dehydrogenase, reduced nicotinamide adenine dinucleotide (phosphate, quinone) activity, flavoprotein NAD(P)H-quinone reductase activity, quinone reductase activity, reduced NAD(P)H dehydrogenase activity, reduced nicotinamide-adenine dinucleotide (phosphate) dehydrogenase activity Subtypes: GO:0008753, NADH dehydrogenase (quinone) (non-electrogenic) activity [GO:0050136]